formation of quadruple SL/U4/U5/U6 snRNP [GO:0000353] (biological process) Note: Note that this step is analogous to 5' splice site selection in cis-splicing. Definition: Formation of a quadruple snRNP complex composed of the spliced leader (SL) RNA along with the U4/U6-U5 tri-snRNP complex. Interactions that may facilitate this include a duplex between the SL and U6 RNAs and interactions between the U5 RNA and the exon sequence at the 5' splice site within the SL RNA. Relationships: is a type of GO:0022618; is part of mRNA trans splicing, SL addition [GO:0045291] Sources: GOC:krc, ISBN:0879695897